{
  "gene_name": "PiggyBac transposable element-derived protein 3",
  "gene": "UniProtKB:Q8N328",
  "gene_symbol": "PGBD3",
  "term_label": "Unknown biological process",
  "term_id": "UNKNOWN:0002"
}